{
  "gene_symbol": "MAPKAPK5",
  "term_id": "GO:0005737",
  "term_label": "cytoplasm",
  "gene_name": "MAP kinase-activated protein kinase 5",
  "gene": "UniProtKB:Q8IW41"
}